{
  "term_id": "GO:0004879",
  "gene_symbol": "ESRRB",
  "term_label": "nuclear receptor activity",
  "gene": "UniProtKB:O95718",
  "gene_name": "Steroid hormone receptor ERR2"
}